{
  "gene_symbol": "CXCL6",
  "gene": "UniProtKB:P80162",
  "term_label": "inflammatory response",
  "gene_name": "C-X-C motif chemokine 6",
  "term_id": "GO:0006954"
}